microtubule associated complex [GO:0005875] (cellular component) Subtypes: GO:0005869, GO:0005871, katanin complex [GO:0008352], GO:0030286, Tea1 cell-end complex [GO:0031500], chromosome passenger complex [GO:0032133], HAUS complex [GO:0070652] Relationships: is a type of protein-containing complex [GO:0032991]; is part of microtubule cytoskeleton [GO:0015630] Sources: GOC:jl Definition: Any multimeric complex connected to a microtubule.